{
  "term_id": "GO:0005737",
  "term_label": "cytoplasm",
  "gene_name": "Protein DDI1 homolog 2",
  "gene_symbol": "DDI2",
  "gene": "UniProtKB:Q5TDH0"
}